thyroid hormone metabolic process [GO:0042403] (biological process) Relationships: is a type of modified amino acid metabolic process [GO:0006575]; is a type of phenol-containing compound metabolic process [GO:0018958]; is a type of hormone metabolic process [GO:0042445] Definition: The chemical reactions and pathways involving any of the compounds secreted by the thyroid gland, largely thyroxine and triiodothyronine. Subtypes: thyroid hormone generation [GO:0006590], thyroid hormone catabolic process [GO:0042404] Also known as: thyroid hormone metabolism Sources: GOC:jl, ISBN:0198506732